{
  "gene_symbol": "GNG5B",
  "gene": "UniProtKB:A0A804HLA8",
  "term_id": "GO:0005834",
  "term_label": "heterotrimeric G-protein complex",
  "gene_name": "Guanine nucleotide-binding protein G(I)_G(S)_G(O) subunit gamma-5B"
}